{
  "gene_symbol": "TBC1D17",
  "gene": "UniProtKB:Q9HA65",
  "term_id": "GO:0005096",
  "gene_name": "TBC1 domain family member 17",
  "term_label": "GTPase activator activity"
}